{
  "term_label": "plasma membrane",
  "term_id": "GO:0005886",
  "gene": "UniProtKB:Q8NGS6",
  "gene_symbol": "OR13C3",
  "gene_name": "Olfactory receptor 13C3"
}